oxidoreductase activity, acting on CH-OH group of donors [GO:0016614] (molecular function) Definition: Catalysis of an oxidation-reduction (redox) reaction in which a CH-OH group act as a hydrogen or electron donor and reduces a hydrogen or electron acceptor. Sources: GOC:ai Also known as: oxidoreductase activity, acting on the CH-OH group of donors, other acceptors Relationships: is a type of oxidoreductase activity [GO:0016491] Subtypes: GO:0004344, lactate dehydrogenase activity [GO:0004457], choline dehydrogenase activity [GO:0008812], malate dehydrogenase activity [GO:0016615], oxidoreductase activity, acting on the CH-OH group of donors, NAD or NADP as acceptor [GO:0016616], oxidoreductase activity, acting on the CH-OH group of donors, cytochrome as acceptor [GO:0016898], oxidoreductase activity, acting on the CH-OH group of donors, oxygen as acceptor [GO:0016899], oxidoreductase activity, acting on the CH-OH group of donors, quinone or similar compound as acceptor [GO:0016901], 1-phenylethanol dehydrogenase activity [GO:0018449], glycolate dehydrogenase activity [GO:0019154], hexitol dehydrogenase activity [GO:0031320], pyranose dehydrogenase (acceptor) activity [GO:0033718], (2R)-oxo-acid reductase activity [GO:0033719], (S)-mandelate dehydrogenase activity [GO:0033720], glucoside 3-dehydrogenase activity [GO:0033757], versicolorin reductase activity [GO:0042469], GO:0045703, (R)-pantolactone dehydrogenase (flavin) activity [GO:0047060], glucose-fructose oxidoreductase activity [GO:0047061], GO:0047545, 3-hydroxycyclohexanone dehydrogenase activity [GO:0047564], GO:0047645, GO:0047735, GO:0047833, GO:0047843, glycerol dehydrogenase (acceptor) activity [GO:0047955], hydroxyacid-oxoacid transhydrogenase activity [GO:0047988], lactate-malate transhydrogenase activity [GO:0050042], GO:0050238, sorbose dehydrogenase activity [GO:0050288], GO:0051990, glucose-6-phosphate dehydrogenase (coenzyme F420) activity [GO:0052749], propan-2-ol:coenzyme F420 oxidoreductase activity [GO:0052753], GO:0052755, leukotriene B4 12-hydroxy dehydrogenase activity [GO:0097257], 20-hydroxy-leukotriene B4 omega oxidase activity [GO:0097258], (R)-mandelate dehydrogenase activity [GO:0097620]